{
  "gene": "UniProtKB:P15918",
  "term_id": "GO:0002331",
  "term_label": "pre-B cell allelic exclusion",
  "gene_name": "V(D)J recombination-activating protein 1",
  "gene_symbol": "RAG1"
}